{
  "gene_name": "BMP_retinoic acid-inducible neural-specific protein 2",
  "term_id": "UNKNOWN:0001",
  "gene": "UniProtKB:Q9C0B6",
  "gene_symbol": "BRINP2",
  "term_label": "Unknown molecular function"
}